epidermal growth factor receptor binding [GO:0005154] (molecular function) Relationships: is_a growth factor receptor binding [GO:0070851] Sources: GOC:ai Definition: Binding to an epidermal growth factor receptor. Also known as: EGF receptor binding, EGFR binding, TGF-alpha receptor binding, TGFalpha receptor binding, transforming growth factor alpha receptor binding, EGF, EGF receptor ligand, epidermal growth factor, epidermal growth factor receptor ligand, transforming growth factor alpha, transforming growth factor alpha receptor ligand